regulation of protein oxidation [GO:1904806] (biological process) Subtypes: negative regulation of protein oxidation [GO:1904807], positive regulation of protein oxidation [GO:1904808] Also known as: regulation of protein amino acid oxidation Relationships: is_a regulation of protein modification process [GO:0031399]; regulates protein oxidation [GO:0018158] References: PMID:22719267 Sources: GOC:TermGenie, GO_REF:0000058 Definition: Any process that modulates the frequency, rate or extent of protein oxidation.